phosphatidylethanolamine binding [GO:0008429] (molecular function) Definition: Binding to a phosphatidylethanolamine, a class of glycerophospholipids in which a phosphatidyl group is esterified to the hydroxyl group of ethanolamine. Sources: ISBN:0198506732 Relationships: is a type of phospholipid binding [GO:0005543]